{
  "term_id": "GO:0005814",
  "gene_symbol": "CEP83",
  "term_label": "centriole",
  "gene": "UniProtKB:Q9Y592",
  "gene_name": "Centrosomal protein of 83 kDa"
}